{
  "term_id": "UNKNOWN:0002",
  "term_label": "Unknown biological process",
  "gene_name": "Protein C3orf33",
  "gene": "UniProtKB:Q6P1S2",
  "gene_symbol": "C3orf33"
}